{
  "gene": "UniProtKB:P16403",
  "term_label": "negative regulation of DNA recombination",
  "gene_symbol": "H1-2",
  "gene_name": "Histone H1.2",
  "term_id": "GO:0045910"
}